{
  "term_id": "GO:0070765",
  "gene_name": "Gamma-secretase subunit PEN-2",
  "term_label": "gamma-secretase complex",
  "gene_symbol": "PSENEN",
  "gene": "UniProtKB:Q9NZ42"
}